{
  "gene_name": "Carcinoembryonic antigen-related cell adhesion molecule 19",
  "gene": "UniProtKB:Q7Z692",
  "term_id": "UNKNOWN:0001",
  "term_label": "Unknown molecular function",
  "gene_symbol": "CEACAM19"
}